{
  "term_label": "UDP-N-acetylglucosamine transferase complex",
  "gene_symbol": "UGT3A1",
  "term_id": "GO:0043541",
  "gene": "UniProtKB:Q6NUS8",
  "gene_name": "UDP-glucuronosyltransferase 3A1"
}